{
  "term_label": "transmembrane signaling receptor activity",
  "gene_name": "VPS10 domain-containing receptor SorCS1",
  "gene_symbol": "SORCS1",
  "term_id": "GO:0004888",
  "gene": "UniProtKB:Q8WY21"
}